{
  "gene_symbol": "OR4C5",
  "term_label": "plasma membrane",
  "term_id": "GO:0005886",
  "gene": "UniProtKB:Q8NGB2",
  "gene_name": "Olfactory receptor 4C5"
}